arabinose:proton symporter activity [GO:0015518] (molecular function) Sources: TC:2.A.1.1.2 Also known as: arabinose efflux permease activity, arabinose efflux transmembrane transporter activity, arabinose:hydrogen symporter activity Definition: Enables the transfer of a solute or solutes from one side of a membrane to the other according to the reaction: arabinose(out) + H+(out) = arabinose(in) + H+(in). Relationships: is a type of carbohydrate:proton symporter activity [GO:0005351]; is_a arabinose transmembrane transporter activity [GO:0042900]